ganglioside GM2 binding [GO:1905574] (molecular function) Definition: Binding to ganglioside GM2. Relationships: is a type of carboxylic acid binding [GO:0031406]; is a type of ganglioside binding [GO:0035594] References: PMID:1454804 Sources: GOC:TermGenie, GO_REF:0000067